{
  "term_label": "Unknown biological process",
  "gene": "UniProtKB:Q8NHX4",
  "term_id": "UNKNOWN:0002",
  "gene_symbol": "SPATA3",
  "gene_name": "Spermatogenesis-associated protein 3"
}